{
  "gene": "UniProtKB:Q96L14",
  "gene_name": "Cep170-like protein",
  "term_id": "UNKNOWN:0002",
  "gene_symbol": "CEP170P1",
  "term_label": "Unknown biological process"
}